{
  "term_id": "GO:0048255",
  "gene": "UniProtKB:Q8IYX4",
  "gene_name": "Dead end protein homolog 1",
  "gene_symbol": "DND1",
  "term_label": "mRNA stabilization"
}